{
  "term_id": "GO:0005634",
  "gene": "UniProtKB:P40424",
  "gene_symbol": "PBX1",
  "gene_name": "Pre-B-cell leukemia transcription factor 1",
  "term_label": "nucleus"
}